{
  "gene": "UniProtKB:Q2M1P5",
  "term_id": "GO:0005737",
  "term_label": "cytoplasm",
  "gene_symbol": "KIF7",
  "gene_name": "Kinesin-like protein KIF7"
}